{
  "gene_symbol": "PIK3R4",
  "term_label": "protein serine/threonine kinase activity",
  "gene_name": "Phosphoinositide 3-kinase regulatory subunit 4",
  "term_id": "GO:0004674",
  "gene": "UniProtKB:Q99570"
}